{
  "gene_name": "Peptidyl-prolyl cis-trans isomerase FKBP7",
  "term_id": "UNKNOWN:0001",
  "gene": "UniProtKB:Q9Y680",
  "gene_symbol": "FKBP7",
  "term_label": "Unknown molecular function"
}